{
  "gene_symbol": "RAI1",
  "gene": "UniProtKB:Q7Z5J4",
  "term_label": "regulation of transcription by RNA polymerase II",
  "gene_name": "Retinoic acid-induced protein 1",
  "term_id": "GO:0006357"
}